{
  "gene": "UniProtKB:O15243",
  "gene_name": "Leptin receptor gene-related protein",
  "gene_symbol": "LEPROT",
  "term_id": "GO:0005768",
  "term_label": "endosome"
}